{
  "gene_symbol": "CCR7",
  "term_label": "cell chemotaxis",
  "gene_name": "C-C chemokine receptor type 7",
  "term_id": "GO:0060326",
  "gene": "UniProtKB:P32248"
}